{
  "gene_name": "Cerberus",
  "gene_symbol": "CER1",
  "gene": "UniProtKB:O95813",
  "term_id": "GO:0035582",
  "term_label": "sequestering of BMP in extracellular matrix"
}